epicardium-derived cardiac fibroblast cell development [GO:0060939] (biological process) Definition: The process whose specific outcome is the progression of an epicardial-derived cardiac fibroblast over time, from its formation to the mature state. A epicardial-derived cardiac fibroblast is a connective tissue cell of the heart that arises from the epicardium and secretes an extracellular matrix rich in collagen and other macromolecules. Sources: GOC:mtg_heart Relationships: is a type of cardiac fibroblast cell development [GO:0060936]; is part of GO:0060938